{
  "gene": "UniProtKB:Q6ZTI6",
  "gene_name": "Refilin-A",
  "gene_symbol": "RFLNA",
  "term_id": "GO:0048705",
  "term_label": "skeletal system morphogenesis"
}